odontogenesis of dentin-containing tooth [GO:0042475] (biological process) Relationships: is a type of odontogenesis [GO:0042476] Note: Note that placoid scales found in the cartilaginous fishes presumably develop through the same processes, but are found on the dermis, rather than in the mouth or pharynx. See Wikipedia:Placoid_scale#Placoid_scales. Definition: The process whose specific outcome is the progression of a dentin-containing tooth over time, from its formation to the mature structure. A dentin-containing tooth is a hard, bony organ borne on the jaw or other bone of a vertebrate, and is composed mainly of dentin, a dense calcified substance, covered by a layer of enamel. Also known as: odontogeny, odontosis, tooth development, odontogenesis of dentine-containing teeth, odontogenesis of dentine-containing tooth Subtypes: GO:0097186, dentinogenesis [GO:0097187] Regulation: regulated by regulation of odontogenesis of dentin-containing tooth [GO:0042487]; positively regulated by positive regulation of odontogenesis of dentin-containing tooth [GO:0042488]; negatively regulated by negative regulation of odontogenesis of dentin-containing tooth [GO:0042489] References: PMID:10333884, PMID:15355794 Sources: GOC:cjm, GOC:mah, GOC:mtg_sensu